GDP-4-dehydro-6-deoxy-D-mannose reductase activity [GO:0033705] (molecular function) Note: Note that this enzyme differs from EC:1.1.1.187, GDP-4-dehydro-D-rhamnose reductase, in that the only product formed is GDP-D-rhamnose (GDP-6-deoxy-D-mannose). Sources: EC:1.1.1.281 Definition: Catalysis of the reaction: GDP-6-deoxy-D-mannose + NAD(P)+ = GDP-4-dehydro-6-deoxy-D-mannose + NAD(P)H + H+. Also known as: GDP-4-keto-6-deoxy-D-mannose reductase activity, GDP-6-deoxy-D-lyxo-4-hexulose reductase activity, GDP-6-deoxy-D-mannose:NAD(P)+ 4-oxidoreductase (D-rhamnose-forming) activity, Rmd Relationships: is a type of oxidoreductase activity, acting on the CH-OH group of donors, NAD or NADP as acceptor [GO:0016616]